{
  "gene": "UniProtKB:P0C0E4",
  "gene_name": "Ras-related protein Rab-40A-like",
  "gene_symbol": "RAB40AL",
  "term_id": "GO:0006887",
  "term_label": "exocytosis"
}